{
  "gene": "UniProtKB:O14929",
  "gene_symbol": "HAT1",
  "gene_name": "Histone acetyltransferase type B catalytic subunit",
  "term_id": "UNKNOWN:0002",
  "term_label": "Unknown biological process"
}